{
  "gene": "UniProtKB:Q6UXF7",
  "gene_name": "C-type lectin domain family 18 member B",
  "gene_symbol": "CLEC18B",
  "term_label": "polysaccharide binding",
  "term_id": "GO:0030247"
}